{
  "term_id": "GO:0003777",
  "gene_name": "Kinesin-like protein KIF21B",
  "term_label": "microtubule motor activity",
  "gene": "UniProtKB:O75037",
  "gene_symbol": "KIF21B"
}